ecdysteroid 22-kinase activity [GO:0106389] (molecular function) Definition: Catalysis of the reaction: an ecdysteroid + ATP = an ecdysteroid 22-phosphate + ADP + H+. Relationships: is a type of GO:0016301 References: PMID:16899460 Sources: RHEA:67972 Also known as: EcKinase